{
  "gene": "UniProtKB:Q86UE4",
  "gene_symbol": "MTDH",
  "term_label": "regulation of transcription by RNA polymerase II",
  "gene_name": "Protein LYRIC",
  "term_id": "GO:0006357"
}